{
  "gene_name": "Solute carrier organic anion transporter family member 4C1",
  "term_id": "GO:0016323",
  "gene_symbol": "SLCO4C1",
  "gene": "UniProtKB:Q6ZQN7",
  "term_label": "basolateral plasma membrane"
}